{
  "gene_name": "Probable phospholipid-transporting ATPase IM",
  "gene": "UniProtKB:Q8TF62",
  "gene_symbol": "ATP8B4",
  "term_label": "ATPase-coupled intramembrane lipid transporter activity",
  "term_id": "GO:0140326"
}